{
  "gene": "UniProtKB:Q9UGM1",
  "term_id": "GO:1904315",
  "gene_name": "Neuronal acetylcholine receptor subunit alpha-9",
  "gene_symbol": "CHRNA9",
  "term_label": "transmitter-gated monoatomic ion channel activity involved in regulation of postsynaptic membrane potential"
}